pyrimidine deoxyribonucleoside monophosphate biosynthetic process [GO:0009177] (BP) Sources: GOC:go_curators, ISBN:0198506732 Relationships: is a type of GO:0009130; is a type of deoxyribonucleoside monophosphate biosynthetic process [GO:0009157]; is a type of pyrimidine deoxyribonucleoside monophosphate metabolic process [GO:0009176] Also known as: pyrimidine deoxyribonucleoside monophosphate anabolism, pyrimidine deoxyribonucleoside monophosphate biosynthesis, pyrimidine deoxyribonucleoside monophosphate formation, pyrimidine deoxyribonucleoside monophosphate synthesis Definition: The chemical reactions and pathways resulting in the formation of pyrimidine deoxynucleoside monophosphate, a compound consisting of a pyrimidine base linked to a deoxyribose sugar esterified with phosphate on the sugar. Subtypes: dUMP biosynthetic process [GO:0006226], dTMP biosynthetic process [GO:0006231], GO:0046064